{
  "gene_name": "Dynein axonemal heavy chain 3",
  "gene_symbol": "DNAH3",
  "term_id": "GO:0036156",
  "term_label": "inner dynein arm",
  "gene": "UniProtKB:Q8TD57"
}